{
  "gene_symbol": "KIF20A",
  "term_id": "GO:0005871",
  "term_label": "kinesin complex",
  "gene": "UniProtKB:O95235",
  "gene_name": "Kinesin-like protein KIF20A"
}